{
  "term_label": "Unknown biological process",
  "gene_symbol": "TBATA",
  "term_id": "UNKNOWN:0002",
  "gene": "UniProtKB:Q96M53",
  "gene_name": "Protein TBATA"
}